{
  "gene_name": "S-adenosyl-L-methionine-dependent tRNA 4-demethylwyosine synthase TYW1B",
  "gene_symbol": "TYW1B",
  "term_label": "Unknown molecular function",
  "gene": "UniProtKB:Q6NUM6",
  "term_id": "UNKNOWN:0001"
}